{
  "gene_name": "Gamma-2-syntrophin",
  "term_label": "dystrophin-associated glycoprotein complex",
  "gene": "UniProtKB:Q9NY99",
  "term_id": "GO:0016010",
  "gene_symbol": "SNTG2"
}